dendrite terminus [GO:0044292] (cellular component) Sources: GOC:jl, NIF_Subcellular:sao28175134 Subtypes: GO:0044293, GO:0044294, dendritic tuft [GO:0044296], dendritic knob [GO:0098788] Relationships: is a type of cellular anatomical structure [GO:0110165]; is part of GO:0030425 Also known as: dendrite terminal, terminal specialization of a dendrite, dendrite terminal specialization, terminal specialization Definition: A structure at the distal end of a dendrite adapted to carry out a specific function, e.g. dendriole.